{
  "term_label": "nucleus",
  "gene_name": "Putative ubiquitin-conjugating enzyme E2 N-like",
  "gene": "UniProtKB:Q5JXB2",
  "term_id": "GO:0005634",
  "gene_symbol": "UBE2NL"
}